{
  "term_label": "reciprocal meiotic recombination",
  "gene_symbol": "SPO11",
  "term_id": "GO:0007131",
  "gene": "UniProtKB:Q9Y5K1",
  "gene_name": "Meiotic recombination protein SPO11"
}